{
  "term_id": "UNKNOWN:0001",
  "gene_symbol": "IBSP",
  "gene_name": "Bone sialoprotein 2",
  "gene": "UniProtKB:P21815",
  "term_label": "Unknown molecular function"
}